{
  "gene_name": "Taste receptor type 2 member 30",
  "term_id": "GO:0033038",
  "gene": "UniProtKB:P59541",
  "term_label": "bitter taste receptor activity",
  "gene_symbol": "TAS2R30"
}